pericentriolar material [GO:0000242] (cellular component) Definition: A network of small fibers that surrounds the centrioles in cells; contains the microtubule nucleating activity of the centrosome. Sources: GOC:clt, ISBN:0815316194 Relationships: is a type of cellular anatomical structure [GO:0110165]; is part of centrosome [GO:0005813]